10-oxogeraniol oxidoreductase activity [GO:0102969] (molecular function) Definition: Catalysis of the reaction: (6E)-8-oxogeraniol + NADP = (6E)-8-oxogeranial + NADPH + H+. Sources: GOC:pz, RHEA:32615 Relationships: is a type of oxidoreductase activity, acting on the CH-OH group of donors, NAD or NADP as acceptor [GO:0016616]